{
  "term_label": "nucleus",
  "term_id": "GO:0005634",
  "gene": "UniProtKB:E7ETH6",
  "gene_symbol": "ZNF587B",
  "gene_name": "Zinc finger protein 587B"
}